regulation of tumor necrosis factor production [GO:0032680] (biological process) Subtypes: negative regulation of tumor necrosis factor production [GO:0032720], positive regulation of tumor necrosis factor production [GO:0032760] Definition: Any process that modulates the frequency, rate or extent of tumor necrosis factor production. Note: Note that this term refers only to the specific, original 'tumor necrosis factor' protein (TNF) and not other members of the tumor necrosis factor superfamily (those with the gene symbol root 'TNFSF'). Also known as: regulation of TNF production, regulation of TNF-alpha production, regulation of cachectin production, regulation of tumor necrosis factor-alpha production, regulation of tumor necrosis factor biosynthetic process, regulation of tumor necrosis factor secretion Relationships: is a type of GO:1903555; regulates tumor necrosis factor production [GO:0032640] References: PMID:10891884, PMID:15560120 Sources: GOC:mah